{
  "term_label": "chromatin binding",
  "gene_symbol": "TSPY10",
  "gene": "UniProtKB:P0CW01",
  "gene_name": "Testis-specific Y-encoded protein 10",
  "term_id": "GO:0003682"
}